{
  "gene_name": "Beta-adrenergic receptor kinase 1",
  "term_id": "GO:0001664",
  "term_label": "G protein-coupled receptor binding",
  "gene_symbol": "GRK2",
  "gene": "UniProtKB:P25098"
}